cyclin A2-CDK1 complex [GO:0097122] (cellular component) Relationships: is a type of cyclin-dependent protein kinase holoenzyme complex [GO:0000307] Definition: A protein complex consisting of cyclin A2 and cyclin-dependent kinase 1 (CDK1). Cyclins are characterized by periodicity in protein abundance throughout the cell cycle. Cyclin-dependent kinases represent a family of serine/threonine protein kinases that become active upon binding to a cyclin regulatory partner. References: PMID:15935619 Sources: GOC:so